{
  "gene_name": "Clathrin heavy chain 2",
  "gene": "UniProtKB:P53675",
  "gene_symbol": "CLTCL1",
  "term_id": "GO:0006898",
  "term_label": "receptor-mediated endocytosis"
}